peripheral mammary gland bud epithelial cell differentiation [GO:0060645] (biological process) Definition: The process in which a relatively unspecialized epithelial cell of the mammary placode becomes an epithelial cell at the periphery of the mammary gland bud. Cells at the periphery of the bud are larger that those of the surrounding epithelium and are arranged concentrically. Relationships: is a type of epithelial cell differentiation involved in mammary gland bud morphogenesis [GO:0060643] References: PMID:12558599 Sources: GOC:dph